heparin binding [GO:0008201] (molecular function) Also known as: heparan sulfate binding Sources: GOC:jl, ISBN:0198506732 Definition: Binding to heparin, a member of a group of glycosaminoglycans found mainly as an intracellular component of mast cells and which consist predominantly of alternating alpha-(1->4)-linked D-galactose and N-acetyl-D-glucosamine-6-sulfate residues. Relationships: is a type of glycosaminoglycan binding [GO:0005539]; is a type of sulfur compound binding [GO:1901681]